{
  "gene_name": "Transketolase-like protein 1",
  "gene": "UniProtKB:P51854",
  "term_label": "Unknown biological process",
  "term_id": "UNKNOWN:0002",
  "gene_symbol": "TKTL1"
}